NAD+-histone H3S10 serine ADP-ribosyltransferase activity [GO:0140817] (molecular function) Relationships: is a type of NAD+-protein-serine ADP-ribosyltransferase activity [GO:0140805] Definition: Catalysis of the transfer of ADP-ribose groups to the serine-10 or an equivalent residue of the N-terminal tail of histone H3. Also known as: NAD+-histone H3-S10 serine ADP-ribosyltransferase activity, NAD+-histone-serine ADP-ribosyltransferase activity (H3-S10 specific) References: PMID:34874266 Note: Comment: Note that the residue position corresponds to the canonical human H3 histone (UniProtKB:P84243); this residue is conserved across all eukaryotes. Residue 1 is the first residue following removal of the initiating Methionine (Met). Note that each histone is encoded by multiple genes, and sequences may vary across different genes within an organism.